{
  "gene": "UniProtKB:P02776",
  "term_label": "cellular response to lipopolysaccharide",
  "term_id": "GO:0071222",
  "gene_name": "Platelet factor 4",
  "gene_symbol": "PF4"
}